{
  "term_label": "Unknown biological process",
  "term_id": "UNKNOWN:0002",
  "gene": "UniProtKB:Q8WV93",
  "gene_symbol": "AFG1L",
  "gene_name": "AFG1-like ATPase"
}